{
  "gene_name": "Anion exchange protein 3",
  "term_label": "plasma membrane",
  "gene_symbol": "SLC4A3",
  "term_id": "GO:0005886",
  "gene": "UniProtKB:P48751"
}